{
  "term_id": "UNKNOWN:0002",
  "gene_name": "Asparagine synthetase domain-containing protein 1",
  "gene_symbol": "ASNSD1",
  "term_label": "Unknown biological process",
  "gene": "UniProtKB:Q9NWL6"
}